negative regulation of peptidyl-L-cysteine S-palmitoylation [GO:1902663] (biological process) Relationships: is_a GO:1902662; is a type of negative regulation of protein lipidation [GO:1903060]; negatively regulates peptidyl-L-cysteine S-palmitoylation [GO:0018230] Definition: Any process that stops, prevents or reduces the frequency, rate or extent of peptidyl-L-cysteine S-palmitoylation. Also known as: down regulation of peptidyl-L-cysteine S-palmitoylation, down regulation of peptidyl-S-palmitoyl-L-cysteine anabolism from peptidyl-cysteine, down regulation of peptidyl-S-palmitoyl-L-cysteine biosynthetic process from peptidyl-cysteine, down regulation of peptidyl-S-palmitoyl-L-cysteine formation from peptidyl-cysteine, down regulation of peptidyl-S-palmitoyl-L-cysteine synthesis from peptidyl-cysteine, down regulation of peptidyl-cysteine S-palmitoylation, down-regulation of peptidyl-L-cysteine S-palmitoylation, down-regulation of peptidyl-S-palmitoyl-L-cysteine anabolism from peptidyl-cysteine, down-regulation of peptidyl-S-palmitoyl-L-cysteine biosynthetic process from peptidyl-cysteine, down-regulation of peptidyl-S-palmitoyl-L-cysteine formation from peptidyl-cysteine, down-regulation of peptidyl-S-palmitoyl-L-cysteine synthesis from peptidyl-cysteine, down-regulation of peptidyl-cysteine S-palmitoylation, downregulation of peptidyl-L-cysteine S-palmitoylation, downregulation of peptidyl-S-palmitoyl-L-cysteine anabolism from peptidyl-cysteine, downregulation of peptidyl-S-palmitoyl-L-cysteine biosynthetic process from peptidyl-cysteine, downregulation of peptidyl-S-palmitoyl-L-cysteine formation from peptidyl-cysteine, downregulation of peptidyl-S-palmitoyl-L-cysteine synthesis from peptidyl-cysteine, downregulation of peptidyl-cysteine S-palmitoylation, negative regulation of peptidyl-S-palmitoyl-L-cysteine anabolism from peptidyl-cysteine, negative regulation of peptidyl-S-palmitoyl-L-cysteine biosynthetic process from peptidyl-cysteine, negative regulation of peptidyl-S-palmitoyl-L-cysteine formation from peptidyl-cysteine, negative regulation of peptidyl-S-palmitoyl-L-cysteine synthesis from peptidyl-cysteine, negative regulation of peptidyl-cysteine S-palmitoylation, inhibition of peptidyl-L-cysteine S-palmitoylation, inhibition of peptidyl-S-palmitoyl-L-cysteine anabolism from peptidyl-cysteine, inhibition of peptidyl-S-palmitoyl-L-cysteine biosynthetic process from peptidyl-cysteine, inhibition of peptidyl-S-palmitoyl-L-cysteine formation from peptidyl-cysteine, inhibition of peptidyl-S-palmitoyl-L-cysteine synthesis from peptidyl-cysteine, inhibition of peptidyl-cysteine S-palmitoylation References: PMID:23444136 Sources: GOC:TermGenie, GO_REF:0000058